Golgi transport complex [GO:0017119] (cellular component) Definition: A multisubunit tethering complex of the CATCHR family (complexes associated with tethering containing helical rods) that has a role in tethering vesicles to the Golgi prior to fusion. Composed of 8 subunits COG1-8. References: PMID:11980916, PMID:20972446, PMID:9792665 Sources: GOC:krc Relationships: is_a vesicle tethering complex [GO:0099023]; is part of Golgi apparatus [GO:0005794] Also known as: COG complex, conserved oligomeric Golgi complex, Sec34/35 complex